{
  "gene_name": "Probable G-protein coupled receptor 132",
  "gene_symbol": "GPR132",
  "gene": "UniProtKB:Q9UNW8",
  "term_label": "Unknown molecular function",
  "term_id": "UNKNOWN:0001"
}